{
  "gene": "UniProtKB:P01286",
  "term_label": "terminal bouton",
  "gene_name": "Somatoliberin",
  "gene_symbol": "GHRH",
  "term_id": "GO:0043195"
}